{
  "gene": "UniProtKB:O15347",
  "gene_name": "High mobility group protein B3",
  "term_label": "Unknown cellular component",
  "gene_symbol": "HMGB3",
  "term_id": "UNKNOWN:0003"
}